spermidine dehydrogenase activity [GO:0050289] (molecular function) Definition: Catalysis of the reaction: spermidine + acceptor + H2O = 1,3-diaminopropane + 4-aminobutanal + reduced acceptor. Sources: EC:1.5.99.6, MetaCyc:SPERMIDINE-DEHYDROGENASE-RXN Also known as: spermidine:(acceptor) oxidoreductase activity, spermidine:acceptor oxidoreductase activity Relationships: is a type of GO:0016645